{
  "term_id": "GO:0050786",
  "term_label": "RAGE receptor binding",
  "gene_name": "Protein S100-A4",
  "gene_symbol": "S100A4",
  "gene": "UniProtKB:P26447"
}